{
  "gene": "UniProtKB:P02647",
  "term_id": "GO:0060228",
  "term_label": "phosphatidylcholine-sterol O-acyltransferase activator activity",
  "gene_name": "Apolipoprotein A-I",
  "gene_symbol": "APOA1"
}